{
  "term_label": "Unknown molecular function",
  "gene": "UniProtKB:Q9GZY1",
  "gene_symbol": "PBOV1",
  "term_id": "UNKNOWN:0001",
  "gene_name": "Prostate and breast cancer overexpressed gene 1 protein"
}